{
  "term_label": "negative regulation of translational initiation in response to stress",
  "gene_symbol": "EIF2AK4",
  "gene": "UniProtKB:Q9P2K8",
  "term_id": "GO:0032057",
  "gene_name": "eIF-2-alpha kinase GCN2"
}